{
  "term_id": "GO:0030890",
  "gene_symbol": "CLCF1",
  "term_label": "positive regulation of B cell proliferation",
  "gene_name": "Cardiotrophin-like cytokine factor 1",
  "gene": "UniProtKB:Q9UBD9"
}